{
  "gene": "UniProtKB:Q30KP8",
  "term_label": "antifungal innate immune response",
  "gene_symbol": "DEFB136",
  "term_id": "GO:0061760",
  "gene_name": "Defensin beta 136"
}